{
  "term_label": "Unknown molecular function",
  "gene_symbol": "TRBV5-8",
  "term_id": "UNKNOWN:0001",
  "gene": "UniProtKB:A0A5A2",
  "gene_name": "T cell receptor beta variable 5-8"
}